{
  "gene": "UniProtKB:Q16667",
  "gene_symbol": "CDKN3",
  "term_id": "GO:0004725",
  "gene_name": "Cyclin-dependent kinase inhibitor 3",
  "term_label": "protein tyrosine phosphatase activity"
}